{
  "gene_symbol": "PACS2",
  "gene": "UniProtKB:Q86VP3",
  "gene_name": "Phosphofurin acidic cluster sorting protein 2",
  "term_id": "UNKNOWN:0003",
  "term_label": "Unknown cellular component"
}